{
  "term_label": "sodium ion transmembrane transport",
  "gene": "UniProtKB:Q9Y3Q4",
  "gene_symbol": "HCN4",
  "term_id": "GO:0035725",
  "gene_name": "Potassium_sodium hyperpolarization-activated cyclic nucleotide-gated channel 4"
}